{
  "term_id": "GO:0030134",
  "gene": "UniProtKB:Q6UWH6",
  "gene_name": "Protein TEX261",
  "gene_symbol": "TEX261",
  "term_label": "COPII-coated ER to Golgi transport vesicle"
}